{
  "term_label": "regulation of glutamate receptor signaling pathway",
  "term_id": "GO:1900449",
  "gene_name": "Major prion protein",
  "gene_symbol": "PRNP",
  "gene": "UniProtKB:P04156"
}